female germ-line stem cell asymmetric division [GO:0048132] (BP) Definition: The self-renewing division of a germline stem cell in the female gonad, to produce a daughter stem cell and a daughter germ cell, which will divide to form the female gametes. Also known as: female germ-line stem cell renewal Relationships: is a type of germline stem cell asymmetric division [GO:0098728]; is part of oogenesis [GO:0048477] Sources: GOC:jid, GOC:mtg_sensu